uterine epithelium development [GO:0035847] (biological process) Sources: GOC:bf, GOC:yaf Also known as: uterus epithelial development Relationships: is a type of oviduct epithelium development [GO:0035846]; is part of uterus development [GO:0060065] Definition: The progression of an epithelium of the uterus over time from its initial formation to the mature structure. An epithelium is a tissue that covers the internal or external surfaces of an anatomical structure.